carotenoid vesicle [GO:0043702] (cellular component) Definition: A tissue-specific cytoplasmic vesicle surrounded by a membrane half-leaflet within which carotenoid pigments are stored. Carotenoid vesicles are synthesized in xanthophores and erythrophore cells and are yellow, orange or red in appearance. Sources: GOC:mh Relationships: is a type of cytoplasmic vesicle [GO:0031410]